{
  "term_label": "translational initiation",
  "term_id": "GO:0006413",
  "gene_symbol": "EIF3C",
  "gene": "UniProtKB:Q99613",
  "gene_name": "Eukaryotic translation initiation factor 3 subunit C"
}